{
  "term_label": "motor neuron axon guidance",
  "gene_name": "E3 ubiquitin-protein ligase ARK2C",
  "gene": "UniProtKB:Q6ZSG1",
  "term_id": "GO:0008045",
  "gene_symbol": "ARK2C"
}